{
  "gene_name": "Transcription factor SOX-3",
  "term_label": "RNA polymerase II cis-regulatory region sequence-specific DNA binding",
  "gene": "UniProtKB:P41225",
  "term_id": "GO:0000978",
  "gene_symbol": "SOX3"
}